negative regulation of lipophagy [GO:1904503] (biological process) Definition: Any process that stops, prevents or reduces the frequency, rate or extent of lipophagy. References: PMID:25383539 Sources: GOC:TermGenie, GOC:autophagy, GOC:dph, GO_REF:0000058 Also known as: down regulation of lipophagy, down-regulation of lipophagy, downregulation of lipophagy, inhibition of lipophagy Relationships: is a type of negative regulation of macroautophagy [GO:0016242]; is a type of regulation of lipophagy [GO:1904502]; negatively regulates lipophagy [GO:0061724]